{
  "term_label": "Unknown cellular component",
  "term_id": "UNKNOWN:0003",
  "gene": "UniProtKB:Q9H4K1",
  "gene_name": "RIB43A-like with coiled-coils protein 2",
  "gene_symbol": "RIBC2"
}